{
  "term_label": "plasma membrane",
  "gene_name": "Olfactory receptor 2J3",
  "gene_symbol": "OR2J3",
  "gene": "UniProtKB:O76001",
  "term_id": "GO:0005886"
}